{
  "gene": "UniProtKB:Q9BQI6",
  "term_id": "UNKNOWN:0001",
  "gene_name": "SMC5-SMC6 complex localization factor protein 1",
  "gene_symbol": "SLF1",
  "term_label": "Unknown molecular function"
}